{
  "term_id": "GO:0009897",
  "gene_symbol": "CLEC4M",
  "term_label": "external side of plasma membrane",
  "gene": "UniProtKB:Q9H2X3",
  "gene_name": "C-type lectin domain family 4 member M"
}